{
  "term_id": "UNKNOWN:0002",
  "gene_name": "GTPase IMAP family member GIMD1",
  "gene_symbol": "GIMD1",
  "gene": "UniProtKB:P0DJR0",
  "term_label": "Unknown biological process"
}